{
  "term_id": "GO:0005667",
  "gene_symbol": "NR4A3",
  "gene": "UniProtKB:Q92570",
  "gene_name": "Nuclear receptor subfamily 4 group A member 3",
  "term_label": "transcription regulator complex"
}